heterotrimeric G-protein complex assembly [GO:1902605] (biological process) Also known as: heterotrimeric G-protein complex formation, heterotrimeric G-protein GTPase, alpha-subunit assembly, heterotrimeric G-protein GTPase, alpha-subunit formation, heterotrimeric G-protein GTPase, beta-subunit assembly, heterotrimeric G-protein GTPase, beta-subunit formation, heterotrimeric G-protein GTPase, gamma-subunit assembly, heterotrimeric G-protein GTPase, gamma-subunit formation, heterotrimeric G-protein GTPase activity assembly, heterotrimeric G-protein GTPase activity formation Relationships: is a type of protein-containing complex assembly [GO:0065003] References: PMID:23637185 Sources: GOC:TermGenie, GOC:dph, GO_REF:0000079 Definition: The aggregation, arrangement and bonding together of a set of components to form a heterotrimeric G-protein complex.